{
  "term_id": "GO:0019005",
  "gene_name": "F-box_WD repeat-containing protein 1A",
  "gene_symbol": "BTRC",
  "gene": "UniProtKB:Q9Y297",
  "term_label": "SCF ubiquitin ligase complex"
}